{
  "term_label": "Unknown molecular function",
  "gene_symbol": "GPD1L",
  "gene": "UniProtKB:Q8N335",
  "term_id": "UNKNOWN:0001",
  "gene_name": "Glycerol-3-phosphate dehydrogenase 1-like protein"
}